phenol kinase activity [GO:0018720] (molecular function) Relationships: is a type of kinase activity [GO:0016301]; is a type of phosphotransferase activity, alcohol group as acceptor [GO:0016773] References: PMID:16980461 Sources: UM-BBD_reactionID:r0155 Definition: Catalysis of the reaction: phenol + X-phosphate = XH + phenylphosphate.